{
  "gene": "UniProtKB:P02042",
  "gene_name": "Hemoglobin subunit delta",
  "term_label": "heme binding",
  "gene_symbol": "HBD",
  "term_id": "GO:0020037"
}